rhombomere 2 structural organization [GO:0021656] (biological process) Sources: GOC:cls, GOC:dgh, GOC:dph, GOC:jid, GO_REF:0000021 Also known as: rhombomere 2 structural organisation Relationships: is a type of GO:0021595; is part of rhombomere 2 morphogenesis [GO:0021655] Definition: The process that contributes to creating the structural organization of rhombomere 2. This process pertains to the physical shaping of a rudimentary structure. Rhombomeres are transverse segments of the developing rhombencephalon. Rhombomeres are lineage restricted, express different genes from one another, and adopt different developmental fates. Rhombomeres are numbered in an anterior to posterior order.